mitochondrial translational termination [GO:0070126] (biological process) Relationships: is a type of translational termination [GO:0006415]; is part of mitochondrial translation [GO:0032543]; BFO_0000066 GO:0005739 Definition: The process resulting in the release of a polypeptide chain from the ribosome in a mitochondrion, usually in response to a termination codon (note that mitochondria use variants of the universal genetic code that differ between different taxa). Also known as: mitochondrial translation termination Sources: GOC:mah, http://mitogenome.org/index.php/Genetic_Code_of_mitochondria